{
  "gene_symbol": "FAM83A",
  "gene": "UniProtKB:Q86UY5",
  "term_id": "GO:0007173",
  "term_label": "epidermal growth factor receptor signaling pathway",
  "gene_name": "Protein FAM83A"
}